beta-sesquiphellandrene synthase activity [GO:0102887] (molecular function) Relationships: is a type of carbon-oxygen lyase activity, acting on phosphates [GO:0016838] Sources: EC:4.2.3.123, GOC:pz Definition: Catalysis of the reaction: 2-trans,6-trans-farnesyl diphosphate = beta-sesquiphellandrene + diphosphoric acid.